{
  "term_id": "UNKNOWN:0003",
  "gene_symbol": "GSTM3",
  "gene_name": "Glutathione S-transferase Mu 3",
  "term_label": "Unknown cellular component",
  "gene": "UniProtKB:P21266"
}